detection of cold stimulus involved in thermoception [GO:0120169] (biological process) References: PMID:21335241 Also known as: sensory detection of cold stimulus during thermoception, sensory transduction of cold stimulus during thermoception, thermoception, sensory detection of cold stimulus, thermoception, sensory transduction of cold stimulus Definition: The series of events in which a cold stimulus is received and converted into a molecular signal as part of thermoception. Relationships: is a type of detection of temperature stimulus involved in thermoception [GO:0050960]; is part of sensory perception of cold stimulus [GO:0062035]